{
  "gene": "UniProtKB:P22310",
  "gene_name": "UDP-glucuronosyltransferase 1A4",
  "term_id": "GO:0001889",
  "term_label": "liver development",
  "gene_symbol": "UGT1A4"
}